{
  "gene_symbol": "OR4C13",
  "gene": "UniProtKB:Q8NGP0",
  "term_label": "olfactory receptor activity",
  "term_id": "GO:0004984",
  "gene_name": "Olfactory receptor 4C13"
}